{
  "gene_name": "Rho GTPase-activating protein 26",
  "term_label": "Unknown biological process",
  "term_id": "UNKNOWN:0002",
  "gene_symbol": "ARHGAP26",
  "gene": "UniProtKB:Q9UNA1"
}